{
  "gene": "UniProtKB:O43707",
  "term_id": "GO:0051015",
  "gene_symbol": "ACTN4",
  "gene_name": "Alpha-actinin-4",
  "term_label": "actin filament binding"
}